cardiac ventricle formation [GO:0003211] (biological process) Sources: GOC:mtg_heart Definition: The developmental process pertaining to the initial formation of a cardiac ventricle from unspecified parts. A cardiac ventricle receives blood from a cardiac atrium and pumps it out of the heart. Relationships: is a type of cardiac chamber formation [GO:0003207]; is part of GO:0003208 Subtypes: cardiac left ventricle formation [GO:0003218], GO:0003219 Regulation: regulated by regulation of cardiac ventricle formation [GO:1904942]; negatively regulated by negative regulation of cardiac ventricle formation [GO:1904943]; positively regulated by positive regulation of cardiac ventricle formation [GO:1904944]